{
  "term_label": "Unknown molecular function",
  "gene_symbol": "HAPSTR2",
  "term_id": "UNKNOWN:0001",
  "gene_name": "HUWE1-associated protein modifying stress responses 2",
  "gene": "UniProtKB:A0A7P0TBJ1"
}